{
  "gene_name": "CUGBP Elav-like family member 6",
  "term_id": "GO:0003729",
  "term_label": "mRNA binding",
  "gene_symbol": "CELF6",
  "gene": "UniProtKB:Q96J87"
}